{
  "term_id": "GO:0051028",
  "gene": "UniProtKB:Q86TG7",
  "term_label": "mRNA transport",
  "gene_name": "Retrotransposon-derived protein PEG10",
  "gene_symbol": "PEG10"
}